{
  "term_id": "GO:0005886",
  "gene_symbol": "KCNH2",
  "gene": "UniProtKB:Q12809",
  "term_label": "plasma membrane",
  "gene_name": "Potassium voltage-gated channel subfamily H member 2"
}